{
  "term_label": "DNA-binding transcription factor activity, RNA polymerase II-specific",
  "gene_symbol": "ZNF813",
  "term_id": "GO:0000981",
  "gene": "UniProtKB:Q6ZN06",
  "gene_name": "Zinc finger protein 813"
}